{
  "gene_name": "Zinc finger protein with KRAB and SCAN domains 8",
  "gene_symbol": "ZKSCAN8",
  "gene": "UniProtKB:Q15776",
  "term_label": "regulation of transcription by RNA polymerase II",
  "term_id": "GO:0006357"
}